{
  "gene_name": "LIM homeobox transcription factor 1-alpha",
  "term_label": "RNA polymerase II transcription regulatory region sequence-specific DNA binding",
  "term_id": "GO:0000977",
  "gene": "UniProtKB:Q8TE12",
  "gene_symbol": "LMX1A"
}